{
  "term_label": "syndecan binding",
  "gene_symbol": "SDCBP",
  "gene": "UniProtKB:O00560",
  "term_id": "GO:0045545",
  "gene_name": "Syntenin-1"
}